{
  "gene_symbol": "CDH3",
  "term_label": "calcium-dependent cell-cell adhesion",
  "gene": "UniProtKB:P22223",
  "term_id": "GO:0016339",
  "gene_name": "Cadherin-3"
}